{
  "gene_symbol": "C6orf47",
  "term_label": "Unknown cellular component",
  "term_id": "UNKNOWN:0003",
  "gene": "UniProtKB:O95873",
  "gene_name": "Uncharacterized protein C6orf47"
}